{
  "gene_symbol": "TRBJ1-6",
  "gene": "UniProtKB:A0A0J9YWX3",
  "term_label": "Unknown biological process",
  "gene_name": "T cell receptor beta joining 1-6",
  "term_id": "UNKNOWN:0002"
}